{
  "term_id": "UNKNOWN:0002",
  "term_label": "Unknown biological process",
  "gene": "UniProtKB:Q7Z403",
  "gene_symbol": "TMC6",
  "gene_name": "Transmembrane channel-like protein 6"
}